{
  "gene_name": "E3 ubiquitin-protein ligase NEURL1",
  "term_label": "positive regulation of long-term neuronal synaptic plasticity",
  "term_id": "GO:0048170",
  "gene_symbol": "NEURL1",
  "gene": "UniProtKB:O76050"
}